{
  "gene_symbol": "MBTPS2",
  "gene_name": "Membrane-bound transcription factor site-2 protease",
  "term_id": "GO:0004222",
  "gene": "UniProtKB:O43462",
  "term_label": "metalloendopeptidase activity"
}